{
  "term_label": "cholesterol homeostasis",
  "gene_name": "Inactive pancreatic lipase-related protein 1",
  "gene_symbol": "PNLIPRP1",
  "term_id": "GO:0042632",
  "gene": "UniProtKB:P54315"
}